{
  "term_id": "GO:0005886",
  "gene_symbol": "ABCC8",
  "gene_name": "ATP-binding cassette sub-family C member 8",
  "gene": "UniProtKB:Q09428",
  "term_label": "plasma membrane"
}